GMP binding [GO:0019002] (molecular function) Definition: Binding to GMP, guanosine monophosphate. Sources: GOC:ai Relationships: is a type of GO:0032561; is a type of GO:0043168